{
  "gene_symbol": "WDCP",
  "term_label": "Unknown cellular component",
  "gene_name": "WD repeat and coiled-coil-containing protein",
  "gene": "UniProtKB:Q9H6R7",
  "term_id": "UNKNOWN:0003"
}